{
  "term_id": "GO:0006357",
  "gene_symbol": "PITX3",
  "gene_name": "Pituitary homeobox 3",
  "term_label": "regulation of transcription by RNA polymerase II",
  "gene": "UniProtKB:O75364"
}